{
  "gene_symbol": "EXOSC6",
  "gene": "UniProtKB:Q5RKV6",
  "term_id": "GO:0071028",
  "gene_name": "Exosome complex component MTR3",
  "term_label": "nuclear mRNA surveillance"
}